stem cell fate specification [GO:0048866] (biological process) Definition: The process in which a cell becomes capable of differentiating autonomously into a stem cell in an environment that is neutral with respect to the developmental pathway. Upon specification, the cell fate can be reversed. Subtypes: GO:0014036 Relationships: is a type of cell fate specification [GO:0001708]; is part of stem cell fate commitment [GO:0048865] Sources: CL:0000034, GOC:isa_complete